{
  "gene_symbol": "NECTIN4",
  "gene_name": "Nectin-4",
  "term_id": "GO:0007157",
  "term_label": "heterophilic cell-cell adhesion",
  "gene": "UniProtKB:Q96NY8"
}